{
  "term_label": "cortical actin cytoskeleton organization",
  "gene_name": "Rho-related GTP-binding protein RhoQ",
  "term_id": "GO:0030866",
  "gene_symbol": "RHOQ",
  "gene": "UniProtKB:P17081"
}